N-acetylmuramoyl-L-alanine amidase activity [GO:0008745] (MF) Relationships: is a type of hydrolase activity, acting on carbon-nitrogen (but not peptide) bonds, in linear amides [GO:0016811]; is a type of peptidoglycan muralytic activity [GO:0061783] Definition: Catalysis of the hydrolysis of the link between N-acetylmuramoyl residues and L-amino acid residues in certain bacterial cell-wall glycopeptides. Also known as: N-acetylmuramic acid L-alanine amidase activity, N-acetylmuramoyl-L-alanine amidase type I, N-acetylmuramoyl-L-alanine amidase type II, N-acetylmuramyl-L-alanine amidase activity, N-acetylmuramylalanine amidase activity, N-acylmuramyl-L-alanine amidase activity, acetylmuramoyl-alanine amidase activity, acetylmuramyl-L-alanine amidase activity, acetylmuramyl-alanine amidase activity References: PMID:22748813 Sources: EC:3.5.1.28